{
  "term_label": "Unknown cellular component",
  "gene_name": "Olfactory receptor 5K2",
  "gene": "UniProtKB:Q8NHB8",
  "gene_symbol": "OR5K2",
  "term_id": "UNKNOWN:0003"
}